conversion of lysyl-tRNA to pyrrolysyl-tRNA [GO:0001720] (biological process) References: PMID:12029131, PMID:12029132, PMID:12121639 Definition: The modification process that results in the conversion of lysine, carried by a specialized lysine-accepting tRNA (possessing a CUA anticodon), to pyrrolysine (a lysine with an amide linkage to a (4R,5R)-4-substituted pyrroline-5-carboxylate). Relationships: is a type of charged-tRNA amino acid modification [GO:0019988]